{
  "term_id": "GO:0070411",
  "gene": "UniProtKB:Q9Y2T1",
  "gene_symbol": "AXIN2",
  "gene_name": "Axin-2",
  "term_label": "I-SMAD binding"
}